{
  "term_label": "mitogen-activated protein kinase binding",
  "gene_name": "MAP kinase-activated protein kinase 2",
  "gene": "UniProtKB:P49137",
  "term_id": "GO:0051019",
  "gene_symbol": "MAPKAPK2"
}